membrane repolarization during SA node cell action potential [GO:0086052] (biological process) Definition: The process in which an SA node cardiac muscle cell membrane potential changes in the direction from the positive membrane potential at the peak of the action potential towards the negative resting potential. Sources: GOC:BHF, GOC:dph, GOC:mtg_cardiac_conduct_nov11 Also known as: membrane repolarization involved in regulation of SA node cardiac muscle cell action potential, membrane repolarization involved in regulation of SAN cardiac muscle cell action potential, membrane repolarization involved in regulation of sinoatrial node cardiac muscle cell action potential, membrane repolarization involved in regulation of sinus node cardiac muscle cell action potential Relationships: is a type of membrane repolarization during cardiac muscle cell action potential [GO:0086013]; is part of SA node cell action potential [GO:0086015]